{
  "term_label": "cytoplasm",
  "gene_name": "Mitochondrial disaggregase",
  "gene": "UniProtKB:Q9H078",
  "term_id": "GO:0005737",
  "gene_symbol": "CLPB"
}